positive regulation of membrane tubulation [GO:1903527] (biological process) References: PMID:18388313 Sources: GOC:TermGenie, GOC:pm, GO_REF:0000058 Definition: Any process that activates or increases the frequency, rate or extent of membrane tubulation. Also known as: positive regulation of plasma membrane tubulation, up regulation of membrane tubulation, up regulation of plasma membrane tubulation, up-regulation of membrane tubulation, up-regulation of plasma membrane tubulation, upregulation of membrane tubulation, upregulation of plasma membrane tubulation, activation of membrane tubulation, activation of plasma membrane tubulation Relationships: is a type of positive regulation of cellular component organization [GO:0051130]; is a type of GO:1903525; positively regulates plasma membrane tubulation [GO:0097320]